molybdenum incorporation into molybdenum-molybdopterin complex [GO:0018315] (biological process) Definition: The incorporation of molybdenum into a molybdenum-molybdopterin complex. Also known as: molybdenum incorporation into metallo-pterin complex Sources: GOC:ai Relationships: is a type of metal incorporation into metallo-molybdopterin complex [GO:0042040]; has part molybdopterin molybdotransferase activity [GO:0061599]